{
  "gene": "UniProtKB:P12830",
  "term_id": "GO:0007416",
  "gene_symbol": "CDH1",
  "gene_name": "Cadherin-1",
  "term_label": "synapse assembly"
}